type I activin receptor binding [GO:0070698] (molecular function) Sources: GOC:BHF, GOC:vk Definition: Binding to a type I activin receptor. Relationships: is a type of activin receptor binding [GO:0070697]